{
  "gene": "UniProtKB:Q04721",
  "term_label": "axon guidance",
  "gene_symbol": "NOTCH2",
  "term_id": "GO:0007411",
  "gene_name": "Neurogenic locus notch homolog protein 2"
}